negative regulation of chemokine (C-X-C motif) ligand 2 production [GO:2000342] (biological process) Sources: GOC:BHF, GOC:mah Relationships: is a type of negative regulation of chemokine production [GO:0032682]; is a type of GO:2000341; negatively regulates GO:0072567 Definition: Any process that stops, prevents or reduces the frequency, rate or extent of chemokine (C-X-C motif) ligand 2 production. Also known as: negative regulation of CXCL2 production, negative regulation of MIP-2 production, negative regulation of MIP2 production, negative regulation of SCYB2 production, inhibition of CCL2 secretion, inhibition of chemokine (C-C motif) ligand 2 secretion, negative regulation of chemokine (C-C motif) ligand 2 secretion